female meiosis chromosome segregation [GO:0016321] (biological process) Relationships: is_a meiotic chromosome segregation [GO:0045132]; is part of female meiotic nuclear division [GO:0007143] Sources: GOC:ai Definition: The cell cycle process in which genetic material, in the form of chromosomes, is organized and then physically separated and apportioned to two or more sets during the meiotic cell cycle in a female. Subtypes: female meiosis chromosome separation [GO:0051309]